alpha4-beta4 integrin-EMILIN-1 complex [GO:0071112] (cellular component) Definition: A protein complex that consists of an alpha4-beta4 integrin complex bound to EMILIN-1 (ElastinMicrofibril Interface Located ProteIN). References: PMID:12456677 Also known as: ITGA4-ITGB4-EMILIN1 complex Relationships: is a type of plasma membrane protein complex [GO:0098797]